{
  "gene_name": "Cullin-2",
  "gene_symbol": "CUL2",
  "term_id": "GO:0019005",
  "gene": "UniProtKB:Q13617",
  "term_label": "SCF ubiquitin ligase complex"
}